{
  "term_id": "GO:0005634",
  "term_label": "nucleus",
  "gene": "UniProtKB:P52738",
  "gene_name": "Zinc finger protein 140",
  "gene_symbol": "ZNF140"
}